ubiquitin-modified histone reader activity [GO:0061649] (molecular function) Also known as: ubiquitin modification-dependent histone binding, ubiquitinated histone binding Definition: A histone reader that recognizes a histone bearing a ubiquinated lysine residue. Relationships: is a type of GO:0140036; is a type of histone reader activity [GO:0140566] References: PMID:24526689